paracellular transport [GO:0160184] (biological process) Relationships: is a type of transport [GO:0006810] Definition: The directed movement of substance through the space in between adjacent cells, rather than through the cells themselves. References: PMID:28452575 Sources: WIki:Paracellular_transport